{
  "gene_name": "Cysteine desulfurase",
  "gene_symbol": "NFS1",
  "gene": "UniProtKB:Q9Y697",
  "term_id": "GO:0005634",
  "term_label": "nucleus"
}